{
  "term_id": "GO:0043197",
  "gene_name": "Glutamate receptor 1",
  "term_label": "dendritic spine",
  "gene": "UniProtKB:P42261",
  "gene_symbol": "GRIA1"
}